intramembrane lipid transporter activity [GO:0140303] (molecular function) Relationships: is a type of lipid transporter activity [GO:0005319]; BFO_0000050 GO:0034204 Subtypes: phospholipid scramblase activity [GO:0017128], ATPase-coupled intramembrane lipid transporter activity [GO:0140326] Definition: Enables the transport of a lipid from a region of a membrane to a different region on the same membrane. Also known as: translocase activity, flippase activity References: PMID:16828084